{
  "gene": "UniProtKB:O00217",
  "gene_symbol": "NDUFS8",
  "term_label": "mitochondrial electron transport, NADH to ubiquinone",
  "term_id": "GO:0006120",
  "gene_name": "NADH dehydrogenase [ubiquinone] iron-sulfur protein 8, mitochondrial"
}